aspartic-type peptidase activity [GO:0070001] (molecular function) Regulation: positively regulated by positive regulation of aspartic-type peptidase activity [GO:1905247] Definition: Catalysis of the hydrolysis of peptide bonds in a polypeptide chain by a mechanism in which a water molecule bound by the side chains of aspartic residues at the active center acts as a nucleophile. Sources: GOC:mah, https://www.ebi.ac.uk/merops/about/glossary.shtml#CATTYPE Subtypes: aspartic-type endopeptidase activity [GO:0004190] Relationships: is a type of peptidase activity [GO:0008233]